{
  "gene_name": "LETM1 domain-containing protein LETM2, mitochondrial",
  "term_id": "GO:0006851",
  "gene": "UniProtKB:Q2VYF4",
  "gene_symbol": "LETM2",
  "term_label": "mitochondrial calcium ion transmembrane transport"
}